{
  "gene_symbol": "HSPA12B",
  "gene": "UniProtKB:Q96MM6",
  "term_label": "Unknown molecular function",
  "gene_name": "Heat shock 70 kDa protein 12B",
  "term_id": "UNKNOWN:0001"
}